venom-mediated suppression of bradykinin-dependent vasodilation [GO:0140163] (biological process) Definition: A process in which an organism inhibits or disrupts vasodilation via the action of a venom that suppresses bradykinin-dependent signaling. References: PMID:21889567, PMID:31370142 Also known as: venom-mediated vasoconstriction via bradykinin receptor antagonism Relationships: is a type of GO:0044513; is a type of venom-mediated perturbation of blood circulation [GO:0140134]